{
  "term_label": "15-oxoprostaglandin 13-reductase [NAD(P)+] activity",
  "gene_name": "Prostaglandin reductase 2",
  "gene_symbol": "PTGR2",
  "term_id": "GO:0047522",
  "gene": "UniProtKB:Q8N8N7"
}